{
  "gene_name": "Zinc finger protein 48",
  "term_label": "nucleus",
  "gene": "UniProtKB:Q96MX3",
  "term_id": "GO:0005634",
  "gene_symbol": "ZNF48"
}